alpha-1,6-mannosylglycoprotein 4-beta-N-acetylglucosaminyltransferase activity [GO:0047253] (molecular function) Definition: Catalysis of the reaction: N-acetyl-beta-D-glucosaminyl-1,6-beta-D-(N-acetyl-B-glucosaminyl-1,2)-beta-D-mannosyl-R + UDP-N-acetyl-D-glucosamine = N-acetyl-beta-D-glucosaminyl-1,6-beta-D-(N-acetyl-D-glucosaminyl-1,2-beta)-(N-acetyl-D-glucosaminyl-1,4-beta)-D-mannosyl-R + UDP. Sources: EC:2.4.1.201, MetaCyc:2.4.1.201-RXN Also known as: alpha-1,6-mannosyl-glycoprotein 4-beta-N-acetylglucosaminyltransferase activity, mannosyl-glycoprotein beta-1,4-N-acetylglucosaminyl-transferase activity, N-acetylglucosaminyltransferase VI activity, N-glycosyl-oligosaccharide-glycoprotein N-acetylglucosaminyltransferase VI activity, UDP-N-acetyl-D-glucosamine:2,6-bis(N-acetyl-beta-D-glucosaminyl)-alpha-D-mannosyl-glycoprotein 4-beta-N-acetyl-D-glucosaminyltransferase activity, mannosyl-glycoprotein beta-1,4-N-acetylglucosaminyltransferase activity, uridine diphosphoacetylglucosamine-glycopeptide beta-1->4-acetylglucosaminyltransferase VI, uridine diphosphoacetylglucosamine-glycopeptide beta-1->4-acetylglucosaminyltransferase VI activity Relationships: is a type of acetylglucosaminyltransferase activity [GO:0008375]; is_a catalytic activity, acting on a glycoprotein [GO:0140103]